{
  "gene": "UniProtKB:Q8NE28",
  "gene_symbol": "STKLD1",
  "gene_name": "Serine_threonine kinase-like domain-containing protein STKLD1",
  "term_label": "Unknown cellular component",
  "term_id": "UNKNOWN:0003"
}